{
  "gene": "UniProtKB:Q04941",
  "gene_symbol": "PLP2",
  "term_id": "GO:0016020",
  "gene_name": "Proteolipid protein 2",
  "term_label": "membrane"
}